{
  "term_label": "B cell differentiation",
  "gene": "UniProtKB:P10721",
  "gene_symbol": "KIT",
  "term_id": "GO:0030183",
  "gene_name": "Mast_stem cell growth factor receptor Kit"
}